{
  "gene_name": "Protein WFDC9",
  "gene": "UniProtKB:Q8NEX5",
  "term_label": "antibacterial humoral response",
  "gene_symbol": "WFDC9",
  "term_id": "GO:0019731"
}